{
  "term_label": "nucleus",
  "gene_symbol": "NCAPH2",
  "term_id": "GO:0005634",
  "gene_name": "Condensin-2 complex subunit H2",
  "gene": "UniProtKB:Q6IBW4"
}